response to glycoside [GO:1903416] (biological process) Definition: Any process that results in a change in state or activity of a cell or an organism (in terms of movement, secretion, enzyme production, gene expression, etc.) as a result of a glycoside stimulus. Also known as: cellular response to ouabain Subtypes: GO:0046679, GO:0097331, response to doxorubicin [GO:1902520], GO:1902522, GO:1904631 Relationships: is a type of response to oxygen-containing compound [GO:1901700] References: PMID:12027881, PMID:16243970 Sources: GOC:BHF, GOC:TermGenie, GOC:mtg_cardiac_conduct_nov11, GOC:rl, GO_REF:0000071